{
  "gene": "UniProtKB:Q9BRQ0",
  "gene_name": "Pygopus homolog 2",
  "term_id": "UNKNOWN:0003",
  "gene_symbol": "PYGO2",
  "term_label": "Unknown cellular component"
}